{
  "term_id": "GO:0050459",
  "gene_symbol": "ETNPPL",
  "term_label": "ethanolamine-phosphate phospho-lyase activity",
  "gene_name": "Ethanolamine-phosphate phospho-lyase",
  "gene": "UniProtKB:Q8TBG4"
}